{
  "gene": "UniProtKB:P13349",
  "term_label": "RNA polymerase II cis-regulatory region sequence-specific DNA binding",
  "term_id": "GO:0000978",
  "gene_symbol": "MYF5",
  "gene_name": "Myogenic factor 5"
}